diaminobutyrate-pyruvate transaminase activity [GO:0047307] (molecular function) Sources: EC:2.6.1.46, RHEA:12380 Relationships: is a type of GO:0008483 Also known as: diaminobutyrate-pyruvate aminotransferase activity, L-2,4-diaminobutanoate:pyruvate aminotransferase activity, L-diaminobutyric acid transaminase activity, diaminobutyrate--pyruvate aminotransferase activity Definition: Catalysis of the reaction: L-2,4-diaminobutyrate + pyruvate = L-alanine + L-aspartate 4-semialdehyde.